{
  "gene": "UniProtKB:P25021",
  "gene_symbol": "HRH2",
  "gene_name": "Histamine H2 receptor",
  "term_id": "GO:0004969",
  "term_label": "histamine receptor activity"
}